globoside alpha-N-acetylgalactosaminyltransferase activity [GO:0047277] (molecular function) Also known as: Forssman synthase activity, UDP-N-acetyl-D-galactosamine:N-acetyl-D-galactosaminyl-1,3-D-galactosyl-1,4-D-galactosyl-1,4-D-glucosylceramide alpha-N-acetyl-D-galactosaminyltransferase activity, globoside acetylgalactosaminyltransferase activity, uridine diphosphoacetylgalactosamine-globoside alpha-acetylgalactosaminyltransferase activity Sources: EC:2.4.1.88, MetaCyc:2.4.1.88-RXN Definition: Catalysis of the reaction: N-acetyl-D-galactosaminyl-(1,3)-D-galactosyl-(1,4)-D-galactosyl-(1,4)-D-glucosylceramide + UDP-N-acetylgalactosamine = N-acetyl-D-galactosaminyl-N-acetyl-D-galactosaminyl-(1,3)-D-galactosyl-(1,4)-D-galactosyl-(1,4)-D-glucosylceramide + UDP. Relationships: is a type of acetylgalactosaminyltransferase activity [GO:0008376]